{
  "gene": "UniProtKB:Q86WR6",
  "gene_name": "CHD1 helical C-terminal domain containing protein 1",
  "gene_symbol": "CHCT1",
  "term_label": "Unknown biological process",
  "term_id": "UNKNOWN:0002"
}